{
  "term_id": "GO:0048814",
  "gene": "UniProtKB:Q96PU5",
  "gene_name": "E3 ubiquitin-protein ligase NEDD4-like",
  "gene_symbol": "NEDD4L",
  "term_label": "regulation of dendrite morphogenesis"
}